{
  "term_id": "GO:0006511",
  "term_label": "ubiquitin-dependent protein catabolic process",
  "gene_symbol": "PSMD3",
  "gene_name": "26S proteasome non-ATPase regulatory subunit 3",
  "gene": "UniProtKB:O43242"
}